protein homotetramerization [GO:0051289] (biological process) Sources: GOC:go_curators Relationships: is a type of protein homooligomerization [GO:0051260]; is a type of protein tetramerization [GO:0051262] Regulation: regulated by GO:1901093; negatively regulated by negative regulation of protein homotetramerization [GO:1901094]; positively regulated by positive regulation of protein homotetramerization [GO:1901095] Also known as: protein homotetramer assembly, protein homotetramer biosynthesis, protein homotetramer biosynthetic process, protein homotetramer formation Definition: The formation of a protein homotetramer, a macromolecular structure consisting of four noncovalently associated identical subunits.